{
  "gene": "UniProtKB:Q969R2",
  "term_id": "GO:0005829",
  "gene_symbol": "OSBP2",
  "gene_name": "Oxysterol-binding protein 2",
  "term_label": "cytosol"
}